{
  "gene_symbol": "PPP2R5C",
  "gene_name": "Serine_threonine-protein phosphatase 2A 56 kDa regulatory subunit gamma isoform",
  "term_id": "GO:0005829",
  "gene": "UniProtKB:Q13362",
  "term_label": "cytosol"
}